{
  "gene_symbol": "TEKT3",
  "gene": "UniProtKB:Q9BXF9",
  "term_label": "Unknown molecular function",
  "term_id": "UNKNOWN:0001",
  "gene_name": "Tektin-3"
}